{
  "gene_name": "Putative olfactory receptor 5AK3",
  "gene": "UniProtKB:Q8NH89",
  "gene_symbol": "OR5AK3P",
  "term_label": "sensory perception of smell",
  "term_id": "GO:0007608"
}